mitochondrial nucleoid [GO:0042645] (CC) Sources: GOC:jl Relationships: is a type of nucleoid [GO:0009295]; is a type of intracellular membraneless organelle [GO:0043232]; is part of mitochondrial matrix [GO:0005759] Definition: The region of a mitochondrion to which the DNA is confined.